{
  "gene": "UniProtKB:Q8TD55",
  "term_id": "UNKNOWN:0001",
  "gene_symbol": "PLEKHO2",
  "gene_name": "Pleckstrin homology domain-containing family O member 2",
  "term_label": "Unknown molecular function"
}